{
  "gene": "UniProtKB:Q9ULZ9",
  "term_label": "collagen catabolic process",
  "gene_symbol": "MMP17",
  "term_id": "GO:0030574",
  "gene_name": "Matrix metalloproteinase-17"
}